{
  "term_id": "UNKNOWN:0002",
  "gene": "UniProtKB:Q8IZQ5",
  "gene_symbol": "SELENOH",
  "gene_name": "Selenoprotein H",
  "term_label": "Unknown biological process"
}